{
  "term_id": "GO:0050806",
  "gene": "UniProtKB:Q9H4D0",
  "gene_symbol": "CLSTN2",
  "term_label": "positive regulation of synaptic transmission",
  "gene_name": "Calsyntenin-2"
}